positive regulation of insulin-like growth factor receptor signaling pathway [GO:0043568] (biological process) Also known as: positive regulation of IGF receptor signaling pathway, positive regulation of IGF receptor signalling pathway, positive regulation of insulin-like growth factor receptor signalling pathway, up regulation of insulin-like growth factor receptor signaling pathway, up-regulation of insulin-like growth factor receptor signaling pathway, upregulation of insulin-like growth factor receptor signaling pathway, activation of insulin-like growth factor receptor signaling pathway, stimulation of insulin-like growth factor receptor signaling pathway Sources: GOC:bf Definition: Any process that increases the frequency, rate or extent of insulin-like growth factor receptor signaling. Relationships: is a type of positive regulation of signal transduction [GO:0009967]; is a type of regulation of insulin-like growth factor receptor signaling pathway [GO:0043567]; positively regulates insulin-like growth factor receptor signaling pathway [GO:0048009]